{
  "gene_name": "Engulfment and cell motility protein 2",
  "gene_symbol": "ELMO2",
  "term_label": "cell motility",
  "gene": "UniProtKB:Q96JJ3",
  "term_id": "GO:0048870"
}